ISG15 ligase activity [GO:0061662] (molecular function) Definition: Catalysis of the transfer of a ISG15 to a substrate protein via the reaction X-ISG15 + S = X + S-ISG15, where X is either an E2 or E3 enzyme, the X-ISG15 linkage is a thioester bond, and the S-ISG15 linkage is an isopeptide bond between the C-terminal amino acid of ISG15 and the epsilon-amino group of lysine residues in the substrate. Sources: GOC:dph Also known as: E3 Relationships: is a type of ISG15 transferase activity [GO:0042296]; is a type of ubiquitin-like protein ligase activity [GO:0061659]